{
  "gene_symbol": "DIO3",
  "term_id": "GO:0042403",
  "gene": "UniProtKB:P55073",
  "gene_name": "Thyroxine 5-deiodinase",
  "term_label": "thyroid hormone metabolic process"
}